{
  "gene_symbol": "EFCAB6",
  "term_label": "Unknown biological process",
  "term_id": "UNKNOWN:0002",
  "gene": "UniProtKB:Q5THR3",
  "gene_name": "EF-hand calcium-binding domain-containing protein 6"
}